sterol import [GO:0035376] (biological process) Definition: The directed movement of a sterol into a cell or organelle. Sterols are steroids with one or more hydroxyl groups and a hydrocarbon side-chain in the molecule. References: PMID:19793923 Sources: GOC:bf Also known as: sterol influx, sterol uptake Relationships: is a type of GO:0015918 Regulation: regulated by GO:2000909; RO_0002212 by GO:2000910; positively regulated by positive regulation of sterol import [GO:2000911]